guanylate cyclase activity [GO:0004383] (molecular function) Sources: EC:4.6.1.2 Relationships: is a type of cyclase activity [GO:0009975]; is a type of phosphorus-oxygen lyase activity [GO:0016849]; is part of cGMP biosynthetic process [GO:0006182] Also known as: guanylyl cyclase activity, receptor guanylate cyclase activity, GTP diphosphate-lyase (cyclizing) activity, GTP diphosphate-lyase (cyclizing; 3',5'-cyclic-GMP-forming) activity, guanyl cyclase activity Definition: Catalysis of the reaction: GTP = 3',5'-cyclic GMP + diphosphate. Regulation: regulated by guanylate cyclase regulator activity [GO:0030249]; positively regulated by GO:0030250; RO_0002212 by GO:0030251; negatively regulated by negative regulation of guanylate cyclase activity [GO:0031283]; positively regulated by positive regulation of guanylate cyclase activity [GO:0031284]